{
  "gene": "UniProtKB:Q5VUM1",
  "term_label": "Unknown molecular function",
  "gene_symbol": "SDHAF4",
  "term_id": "UNKNOWN:0001",
  "gene_name": "Succinate dehydrogenase assembly factor 4, mitochondrial"
}